{
  "gene": "UniProtKB:Q8TAM6",
  "term_id": "GO:0051015",
  "term_label": "actin filament binding",
  "gene_symbol": "ERMN",
  "gene_name": "Ermin"
}